{
  "gene_symbol": "ZMYND10",
  "gene_name": "Zinc finger MYND domain-containing protein 10",
  "term_id": "GO:0036159",
  "gene": "UniProtKB:O75800",
  "term_label": "inner dynein arm assembly"
}